response to lithium ion [GO:0010226] (biological process) Subtypes: GO:0071285 Definition: Any process that results in a change in state or activity of a cell or an organism (in terms of movement, secretion, enzyme production, gene expression, etc.) as a result of a lithium (Li+) ion stimulus. Sources: GOC:tb Relationships: is a type of GO:0010038